tRNA threonylcarbamoyladenosine modification [GO:0002949] (biological process) References: PMID:19287007, PMID:21183954, PMID:23258706 Sources: GOC:imk, GOC:mah Also known as: t6A biosynthesis, t6A biosynthetic process, t6A tRNA modification, threonylcarbamoyladenosine anabolism, threonylcarbamoyladenosine biosynthesis, threonylcarbamoyladenosine biosynthetic process, threonylcarbamoyladenosine formation, threonylcarbamoyladenosine synthesis Subtypes: mitochondrial tRNA threonylcarbamoyladenosine modification [GO:0072670] Relationships: is a type of tRNA modification [GO:0006400]; is_a tRNA threonylcarbamoyladenosine metabolic process [GO:0070525] Definition: The attachment of a carbonyl group and a threonine to the amino group of the adenine residue immediately 3' of the anticodon, in tRNAs that decode ANN codons (where N is any base).